{
  "term_label": "endoplasmic reticulum unfolded protein response",
  "gene_name": "Ubiquitin thioesterase OTU1",
  "gene": "UniProtKB:Q5VVQ6",
  "gene_symbol": "YOD1",
  "term_id": "GO:0030968"
}